{
  "term_label": "autophagosome maturation",
  "term_id": "GO:0097352",
  "gene_symbol": "MAP1LC3B",
  "gene": "UniProtKB:Q9GZQ8",
  "gene_name": "Microtubule-associated proteins 1A_1B light chain 3B"
}